{
  "term_label": "ciliary membrane",
  "gene_name": "EvC complex member EVC",
  "gene": "UniProtKB:P57679",
  "gene_symbol": "EVC",
  "term_id": "GO:0060170"
}